{
  "term_label": "protein ubiquitination",
  "gene_name": "E3 ubiquitin-protein ligase MIB1",
  "gene_symbol": "MIB1",
  "gene": "UniProtKB:Q86YT6",
  "term_id": "GO:0016567"
}